{
  "gene_symbol": "KCTD13",
  "term_id": "GO:0035024",
  "gene": "UniProtKB:Q8WZ19",
  "gene_name": "BTB_POZ domain-containing adapter for CUL3-mediated RhoA degradation protein 1",
  "term_label": "negative regulation of Rho protein signal transduction"
}